{
  "term_id": "GO:0000139",
  "term_label": "Golgi membrane",
  "gene_name": "Galactosylgalactosylxylosylprotein 3-beta-glucuronosyltransferase 2",
  "gene_symbol": "B3GAT2",
  "gene": "UniProtKB:Q9NPZ5"
}